alpha-glucan catabolic process [GO:0030980] (biological process) Also known as: alpha-glucan breakdown, alpha-glucan catabolism, alpha-glucan degradation Sources: GOC:mah Relationships: is a type of glucan catabolic process [GO:0009251]; is a type of alpha-glucan metabolic process [GO:0030978] Definition: The chemical reactions and pathways resulting in the breakdown of alpha-glucans.